{
  "gene_symbol": "MAPK15",
  "gene": "UniProtKB:Q8TD08",
  "gene_name": "Mitogen-activated protein kinase 15",
  "term_id": "GO:0005737",
  "term_label": "cytoplasm"
}